{
  "term_id": "GO:0000045",
  "gene": "UniProtKB:Q9NT62",
  "term_label": "autophagosome assembly",
  "gene_name": "Ubiquitin-like-conjugating enzyme ATG3",
  "gene_symbol": "ATG3"
}